{
  "term_label": "insulin receptor binding",
  "gene_symbol": "GRB10",
  "term_id": "GO:0005158",
  "gene_name": "Growth factor receptor-bound protein 10",
  "gene": "UniProtKB:Q13322"
}